{
  "term_id": "GO:0060090",
  "gene": "UniProtKB:Q99996",
  "gene_symbol": "AKAP9",
  "gene_name": "A-kinase anchor protein 9",
  "term_label": "molecular adaptor activity"
}